{
  "term_id": "UNKNOWN:0003",
  "term_label": "Unknown cellular component",
  "gene_name": "Protein HEG homolog 1",
  "gene": "UniProtKB:Q9ULI3",
  "gene_symbol": "HEG1"
}